{
  "gene": "UniProtKB:P04090",
  "term_label": "Unknown molecular function",
  "term_id": "UNKNOWN:0001",
  "gene_name": "Prorelaxin H2",
  "gene_symbol": "RLN2"
}